{
  "term_id": "GO:0005251",
  "gene": "UniProtKB:Q03721",
  "term_label": "delayed rectifier potassium channel activity",
  "gene_name": "Potassium voltage-gated channel subfamily C member 4",
  "gene_symbol": "KCNC4"
}